{
  "term_id": "GO:0002767",
  "term_label": "immune response-inhibiting cell surface receptor signaling pathway",
  "gene_name": "Killer cell immunoglobulin-like receptor, two Ig domains pseudogene 1",
  "gene_symbol": "KIR2DP1",
  "gene": "UniProtKB:A0A0G2JNF4"
}